{
  "term_id": "GO:0038158",
  "gene": "UniProtKB:Q8N5M9",
  "gene_symbol": "JAGN1",
  "gene_name": "Protein jagunal homolog 1",
  "term_label": "granulocyte colony-stimulating factor signaling pathway"
}